{
  "term_label": "mRNA binding",
  "gene_name": "Small ribosomal subunit protein eS26",
  "gene_symbol": "RPS26",
  "term_id": "GO:0003729",
  "gene": "UniProtKB:P62854"
}